{
  "term_label": "chromatin binding",
  "gene": "UniProtKB:P51531",
  "gene_symbol": "SMARCA2",
  "term_id": "GO:0003682",
  "gene_name": "Probable global transcription activator SNF2L2"
}